{
  "gene_name": "Nuclear pore complex protein Nup88",
  "gene": "UniProtKB:Q99567",
  "term_label": "ribosomal large subunit export from nucleus",
  "gene_symbol": "NUP88",
  "term_id": "GO:0000055"
}